5-methylphenazine-1-carboxylate 1-monooxygenase (NADH) activity [GO:0102169] (molecular function) Definition: Catalysis of the reaction: 5-methyl-phenazine-1-carboxylate + 2 H+ + NADH + O2 = CO2 + H2O + NAD+ + pyocyanin. Also converts phenazine-1-carboxylate into 1-hydroxyphenazine. Also known as: pyocyanin hydroxylase activity Relationships: is_a GO:0016709 References: PMID:11591691 Sources: EC:1.14.13.218